{
  "term_label": "DNA binding",
  "gene": "UniProtKB:Q5SSJ5",
  "term_id": "GO:0003677",
  "gene_name": "Heterochromatin protein 1-binding protein 3",
  "gene_symbol": "HP1BP3"
}